{
  "gene_symbol": "FOXS1",
  "term_label": "DNA-binding transcription factor activity, RNA polymerase II-specific",
  "term_id": "GO:0000981",
  "gene_name": "Forkhead box protein S1",
  "gene": "UniProtKB:O43638"
}